{
  "term_label": "Unknown cellular component",
  "gene": "UniProtKB:Q9UHI5",
  "gene_symbol": "SLC7A8",
  "term_id": "UNKNOWN:0003",
  "gene_name": "Large neutral amino acids transporter small subunit 2"
}